{
  "gene": "UniProtKB:O43791",
  "gene_name": "Speckle-type POZ protein",
  "gene_symbol": "SPOP",
  "term_id": "GO:0005634",
  "term_label": "nucleus"
}